{
  "gene_name": "Origin recognition complex subunit 6",
  "gene": "UniProtKB:Q9Y5N6",
  "term_label": "DNA replication initiation",
  "term_id": "GO:0006270",
  "gene_symbol": "ORC6"
}